{
  "term_id": "GO:0030674",
  "gene_symbol": "LIN7C",
  "term_label": "protein-macromolecule adaptor activity",
  "gene": "UniProtKB:Q9NUP9",
  "gene_name": "Protein lin-7 homolog C"
}